{
  "gene_name": "Helix-loop-helix protein 2",
  "term_label": "Unknown cellular component",
  "term_id": "UNKNOWN:0003",
  "gene": "UniProtKB:Q02577",
  "gene_symbol": "NHLH2"
}